methyltransferase complex [GO:0034708] (cellular component) Definition: A protein complex that possesses methyltransferase activity. Relationships: is a type of GO:1990234; is part of intracellular anatomical structure [GO:0005622] Subtypes: methylosome [GO:0034709], histone methyltransferase complex [GO:0035097], eRF1 methyltransferase complex [GO:0035657], RNA N6-methyladenosine methyltransferase complex [GO:0036396], GO:0043527, methanol-CoM methyltransferase complex [GO:0043853], methylthiol:coenzyme M methyltransferase complex [GO:0044680], DNA methyltransferase complex [GO:0140020], GO:0160130 Sources: GOC:mah